histone H3K27 methyltransferase activity [GO:0046976] (MF) Sources: GOC:ai Subtypes: histone H3K27 trimethyltransferase activity [GO:0140951], histone H3K27 dimethyltransferase activity [GO:0140952], histone H3K27 monomethyltransferase activity [GO:0140953] Note: Comment: Note that the residue position corresponds to the canonical human H3 histone (UniProtKB:P84243); this residue is conserved across all eukaryotes. Residue 1 is the first residue following removal of the initiating Methionine (Met). Note that each histone is encoded by multiple genes, and sequences may vary across different genes within an organism. Also known as: histone H3K27 methylase activity, histone lysine N-methyltransferase activity (H3-K27 specific), histone methylase activity (H3-K27 specific), histone methylase activity (H3-K56 specific), histone methyltransferase activity (H3-K27 specific), histone-H3K27 methyltransferase activity Definition: Catalysis of the reaction: S-adenosyl-L-methionine + histone H3 L-lysine (position 27) = S-adenosyl-L-homocysteine + histone H3 N6-methyl-L-lysine (position 27). This reaction is the addition of a methyl group to the lysine residue at position 27 of the histone H3 protein. Relationships: is a type of protein-lysine N-methyltransferase activity [GO:0016279]; is a type of histone H3 methyltransferase activity [GO:0140938]